{
  "gene_symbol": "NR0B2",
  "term_label": "nuclear receptor binding",
  "gene_name": "Nuclear receptor subfamily 0 group B member 2",
  "term_id": "GO:0016922",
  "gene": "UniProtKB:Q15466"
}